{
  "gene": "UniProtKB:Q8N7X2",
  "term_id": "UNKNOWN:0002",
  "gene_name": "Protein STPG3",
  "gene_symbol": "STPG3",
  "term_label": "Unknown biological process"
}